{
  "term_id": "GO:0070836",
  "gene_name": "Caveolin-2",
  "gene_symbol": "CAV2",
  "gene": "UniProtKB:P51636",
  "term_label": "caveola assembly"
}